interleukin-1, type II receptor binding [GO:0005151] (molecular function) Sources: GOC:ai Also known as: IL-1 type II, interleukin-1, type II receptor ligand Relationships: is a type of interleukin-1 receptor binding [GO:0005149] Definition: Binding to a Type II interleukin-1 receptor.